{
  "gene": "UniProtKB:Q6P1K8",
  "term_label": "transcription factor TFIIH holo complex",
  "term_id": "GO:0005675",
  "gene_symbol": "GTF2H2C",
  "gene_name": "General transcription factor IIH subunit 2-like protein"
}